bacteriocin biosynthetic process [GO:0030152] (biological process) Also known as: bacteriocin anabolism, bacteriocin biosynthesis, bacteriocin formation, bacteriocin synthesis Definition: The chemical reactions and pathways resulting in the formation of a bacteriocin, any of a heterogeneous group of polypeptide antibiotics that are secreted by certain bacterial strains and are able to kill cells of other susceptible (frequently related) strains after adsorption at specific receptors on the cell surface. They include the colicins, and their mechanisms of action vary. Sources: GOC:mah, ISBN:0198506732 Relationships: is a type of toxin biosynthetic process [GO:0009403]; is a type of GO:0030651; is a type of bacteriocin metabolic process [GO:0046224]